phagolysosome [GO:0032010] (cellular component) Also known as: late phagocytic vesicle, late phagosome Subtypes: food vacuole [GO:0020020] Relationships: is a type of secondary lysosome [GO:0005767]; is a type of phagocytic vesicle [GO:0045335] References: PMID:12388753, PMID:14733906 Sources: GOC:mah Definition: A membrane-bounded intracellular vesicle formed by maturation of an early phagosome following the ingestion of particulate material by phagocytosis; during maturation, phagosomes acquire markers of late endosomes and lysosomes.